nerve growth factor signaling pathway [GO:0038180] (biological process) References: PMID:11520933 Sources: GOC:bf Definition: The series of molecular signals initiated by nerve growth factor (NGF) binding to its receptor on the surface of a target cell, and ending with the regulation of a downstream cellular process, e.g. transcription. Note: Nerve growth factor (NGF) binds at least two classes of receptors: the p75 LNGFR (low-affinity nerve growth factor receptor) and TrkA, a transmembrane tyrosine kinase. Also known as: NGF signaling pathway, nerve growth factor signalling pathway Relationships: is a type of neurotrophin signaling pathway [GO:0038179]; BFO_0000050 cellular response to nerve growth factor stimulus [GO:1990090]